{
  "gene": "UniProtKB:P32004",
  "term_label": "neuronal cell body",
  "gene_name": "Neural cell adhesion molecule L1",
  "gene_symbol": "L1CAM",
  "term_id": "GO:0043025"
}